{
  "gene_symbol": "TRGJ1",
  "gene": "UniProtKB:A0A075B6S0",
  "gene_name": "T cell receptor gamma joining 1",
  "term_label": "Unknown cellular component",
  "term_id": "UNKNOWN:0003"
}